positive regulation of short-day photoperiodism, flowering [GO:0048576] (biological process) Relationships: is a type of GO:0048582; is a type of positive regulation of response to stimulus [GO:0048584]; is a type of GO:0048587; positively regulates GO:0048575 Sources: GOC:jid, GOC:pj, ISBN:0582015952, ISBN:0697037754, ISBN:0709408862 Definition: Any process that activates, maintains or increases short-day photoperiodism, where the response associated with the photoperiodism is flowering. Flowering is defined by the switch from the vegetative to the reproductive phase. Also known as: up regulation of short-day photoperiodism, flowering, up-regulation of short-day photoperiodism, flowering, upregulation of short-day photoperiodism, flowering, activation of short-day photoperiodism, flowering, stimulation of short-day photoperiodism, flowering